{
  "term_id": "GO:0004505",
  "term_label": "phenylalanine 4-monooxygenase activity",
  "gene": "UniProtKB:P00439",
  "gene_symbol": "PAH",
  "gene_name": "Phenylalanine-4-hydroxylase"
}